{
  "gene_name": "NADPH-dependent diflavin oxidoreductase 1",
  "term_id": "GO:0016491",
  "term_label": "oxidoreductase activity",
  "gene_symbol": "NDOR1",
  "gene": "UniProtKB:Q9UHB4"
}